{
  "term_label": "Unknown cellular component",
  "term_id": "UNKNOWN:0003",
  "gene_symbol": "ISM1",
  "gene": "UniProtKB:B1AKI9",
  "gene_name": "Isthmin-1"
}